{
  "term_label": "glycine binding",
  "gene_symbol": "GNMT",
  "term_id": "GO:0016594",
  "gene": "UniProtKB:Q14749",
  "gene_name": "Glycine N-methyltransferase"
}